clathrin-coated vesicle cargo loading, AP-3-mediated [GO:0035654] (biological process) References: PMID:12802059, PMID:16162817 Sources: GOC:lb Relationships: is a type of GO:0035652 Also known as: cargo loading into clathrin-coated vesicle, AP-3-mediated Definition: Formation of a macromolecular complex between proteins of the AP-3 adaptor complex and proteins and/or lipoproteins that are going to be transported by a clathrin-coated vesicle. In some cases, the AP-3 complex is a heterotetrameric AP-type membrane coat adaptor complex that, in some organisms, links clathrin to the membrane surface of a vesicle.